{
  "gene": "UniProtKB:P54619",
  "gene_symbol": "PRKAG1",
  "term_id": "GO:0031588",
  "gene_name": "5'-AMP-activated protein kinase subunit gamma-1",
  "term_label": "nucleotide-activated protein kinase complex"
}